{
  "term_id": "GO:0005737",
  "gene": "UniProtKB:Q96AB3",
  "gene_name": "Isochorismatase domain-containing protein 2",
  "gene_symbol": "ISOC2",
  "term_label": "cytoplasm"
}